negative regulation of vitamin D receptor signaling pathway [GO:0070563] (biological process) Definition: Any process that stops, prevents, or reduces the frequency, rate or extent of the vitamin D receptor signaling pathway activity. Also known as: down regulation of vitamin D receptor signaling pathway, down-regulation of vitamin D receptor signaling pathway, downregulation of vitamin D receptor signaling pathway, negative regulation of VDR signaling pathway, negative regulation of VDR signalling pathway, negative regulation vitamin D receptor signalling pathway, inhibition of vitamin D receptor signaling pathway Relationships: is a type of regulation of vitamin D receptor signaling pathway [GO:0070562]; is a type of negative regulation of intracellular signal transduction [GO:1902532]; negatively regulates vitamin D receptor signaling pathway [GO:0070561] Sources: GOC:BHF, GOC:mah